{
  "gene_symbol": "ADGRG6",
  "gene_name": "Adhesion G-protein coupled receptor G6",
  "gene": "UniProtKB:Q86SQ4",
  "term_label": "myelination in peripheral nervous system",
  "term_id": "GO:0022011"
}